{
  "gene_symbol": "BCL6",
  "term_id": "GO:0042127",
  "gene": "UniProtKB:P41182",
  "gene_name": "B-cell lymphoma 6 protein",
  "term_label": "regulation of cell population proliferation"
}